{
  "gene": "UniProtKB:Q96RU8",
  "gene_name": "Tribbles homolog 1",
  "term_id": "GO:0032436",
  "term_label": "positive regulation of proteasomal ubiquitin-dependent protein catabolic process",
  "gene_symbol": "TRIB1"
}